positive regulation of growth factor dependent skeletal muscle satellite cell proliferation [GO:1902728] (biological process) Definition: Any process that activates or increases the frequency, rate or extent of satellite cell proliferation; dependent on specific growth factor activity such as fibroblast growth factors and transforming growth factor beta. References: PMID:23212449 Sources: GOC:TermGenie, GO_REF:0000058 Relationships: is_a positive regulation of skeletal muscle satellite cell proliferation [GO:1902724]